{
  "term_id": "GO:0005634",
  "gene_name": "Protein Red",
  "term_label": "nucleus",
  "gene_symbol": "IK",
  "gene": "UniProtKB:Q13123"
}